{
  "gene": "UniProtKB:O95395",
  "gene_name": "Beta-1,3-galactosyl-O-glycosyl-glycoprotein beta-1,6-N-acetylglucosaminyltransferase 3",
  "gene_symbol": "GCNT3",
  "term_id": "UNKNOWN:0003",
  "term_label": "Unknown cellular component"
}